{
  "term_label": "elastic fiber assembly",
  "gene_name": "EGF-containing fibulin-like extracellular matrix protein 2",
  "gene": "UniProtKB:O95967",
  "gene_symbol": "EFEMP2",
  "term_id": "GO:0048251"
}